Peyer's patch morphogenesis [GO:0061146] (biological process) Sources: GOC:dph Definition: The process in which a Peyer's patch is generated and organized. Peyer's patches are typically found as nodules associated with gut epithelium with distinct internal structures including B- and T-zones for the activation of lymphocytes. Relationships: is a type of GO:0048729; is part of Peyer's patch development [GO:0048541]